{
  "gene_name": "Tumor protein D53",
  "gene": "UniProtKB:Q16890",
  "term_id": "GO:0005737",
  "gene_symbol": "TPD52L1",
  "term_label": "cytoplasm"
}